{
  "gene_symbol": "MARVELD3",
  "gene_name": "MARVEL domain-containing protein 3",
  "term_label": "Unknown cellular component",
  "gene": "UniProtKB:Q96A59",
  "term_id": "UNKNOWN:0003"
}